{
  "gene": "UniProtKB:Q96HC4",
  "gene_name": "PDZ and LIM domain protein 5",
  "term_id": "GO:0007507",
  "term_label": "heart development",
  "gene_symbol": "PDLIM5"
}